{
  "gene_name": "Myelin basic protein",
  "gene": "UniProtKB:P02686",
  "gene_symbol": "MBP",
  "term_id": "UNKNOWN:0001",
  "term_label": "Unknown molecular function"
}